D-alanine gamma-glutamyltransferase activity [GO:0047811] (MF) Relationships: is a type of aminoacyltransferase activity [GO:0016755] Sources: RHEA:23556 Definition: Catalysis of the reaction: D-alanine + L-glutamine = gamma-L-glutamyl-D-alanine + NH4. Also known as: D-alanine g-glutamyltransferase activity